{
  "gene": "UniProtKB:Q5VXU1",
  "term_label": "regulation of sodium ion transport",
  "gene_name": "Sodium_potassium-transporting ATPase subunit beta-1-interacting protein 2",
  "term_id": "GO:0002028",
  "gene_symbol": "NKAIN2"
}